{
  "term_label": "late endosome membrane",
  "gene": "UniProtKB:Q14849",
  "gene_name": "StAR-related lipid transfer protein 3",
  "term_id": "GO:0031902",
  "gene_symbol": "STARD3"
}